{
  "term_label": "mitotic DNA replication preinitiation complex assembly",
  "gene_name": "Cell division control protein 45 homolog",
  "gene_symbol": "CDC45",
  "gene": "UniProtKB:O75419",
  "term_id": "GO:1902977"
}